regulation of eclosion [GO:0007563] (biological process) Definition: Any process that modulates the frequency, rate or extent of the emergence of an insect from a pupa-case or of a larva from an egg. Sources: GOC:go_curators, ISBN:0198600461 Relationships: is a type of regulation of multicellular organismal development [GO:2000026]; regulates eclosion [GO:0007562] Subtypes: GO:0045804, GO:0045805